{
  "term_label": "nucleolus",
  "gene": "UniProtKB:Q9H1J1",
  "gene_name": "Regulator of nonsense transcripts 3A",
  "gene_symbol": "UPF3A",
  "term_id": "GO:0005730"
}